{
  "gene_symbol": "FAM107A",
  "gene": "UniProtKB:O95990",
  "term_id": "GO:0051017",
  "term_label": "actin filament bundle assembly",
  "gene_name": "Actin-associated protein FAM107A"
}